alpha6-beta4 integrin-CD9 complex [GO:0071094] (cellular component) References: PMID:10711425 Relationships: is_a plasma membrane protein complex [GO:0098797] Also known as: ITGA6-ITGB4-CD9 complex Definition: A protein complex that consists of an alpha6-beta4 integrin complex bound to the cell surface protein CD9.